{
  "term_id": "GO:0016197",
  "gene_name": "Intersectin-1",
  "gene_symbol": "ITSN1",
  "gene": "UniProtKB:Q15811",
  "term_label": "endosomal transport"
}